{
  "term_id": "GO:0070374",
  "gene": "UniProtKB:Q9NZC2",
  "gene_name": "Triggering receptor expressed on myeloid cells 2",
  "gene_symbol": "TREM2",
  "term_label": "positive regulation of ERK1 and ERK2 cascade"
}